{
  "gene_name": "Ecto-ADP-ribosyltransferase 3",
  "gene": "UniProtKB:Q13508",
  "term_id": "UNKNOWN:0002",
  "gene_symbol": "ART3",
  "term_label": "Unknown biological process"
}